{
  "term_id": "UNKNOWN:0001",
  "gene_symbol": "A0A0G2JPN4",
  "gene": "UniProtKB:A0A0G2JPN4",
  "term_label": "Unknown molecular function",
  "gene_name": "Uncharacterized protein"
}